chemokine receptor transport within lipid bilayer [GO:0033606] (biological process) Definition: The directed movement of a chemokine receptor within a lipid bilayer. Sources: GOC:mah Also known as: chemokine receptor translocation within membrane Relationships: is a type of protein transport within lipid bilayer [GO:0032594] Subtypes: chemokine receptor transport out of membrane raft [GO:0032600]